{
  "term_id": "GO:0009897",
  "gene_symbol": "LIFR",
  "term_label": "external side of plasma membrane",
  "gene_name": "Leukemia inhibitory factor receptor",
  "gene": "UniProtKB:P42702"
}